dendritic spine maintenance [GO:0097062] (biological process) Regulation: regulated by regulation of dendritic spine maintenance [GO:1902950]; negatively regulated by negative regulation of dendritic spine maintenance [GO:1902951]; positively regulated by positive regulation of dendritic spine maintenance [GO:1902952] Relationships: is a type of cellular component maintenance [GO:0043954]; is a type of dendritic spine organization [GO:0097061] Definition: The organization process that preserves a dendritic spine in a stable functional or structural state. A dendritic spine is a specialized protrusion from a neuronal dendrite and is involved in synaptic transmission. References: PMID:20410104 Sources: GOC:BHF